{
  "term_id": "GO:0000981",
  "gene_symbol": "ZNF728",
  "gene": "UniProtKB:P0DKX0",
  "term_label": "DNA-binding transcription factor activity, RNA polymerase II-specific",
  "gene_name": "Zinc finger protein 728"
}